{
  "gene_name": "Hornerin",
  "term_id": "GO:0061436",
  "gene": "UniProtKB:Q86YZ3",
  "gene_symbol": "HRNR",
  "term_label": "establishment of skin barrier"
}